{
  "gene_name": "Zinc finger protein 354A",
  "term_label": "nucleus",
  "term_id": "GO:0005634",
  "gene": "UniProtKB:O60765",
  "gene_symbol": "ZNF354A"
}